{
  "gene_symbol": "HACE1",
  "term_label": "Golgi organization",
  "gene_name": "E3 ubiquitin-protein ligase HACE1",
  "term_id": "GO:0007030",
  "gene": "UniProtKB:Q8IYU2"
}